{
  "gene_name": "Solute carrier family 2, facilitated glucose transporter member 12",
  "gene": "UniProtKB:Q8TD20",
  "term_label": "D-glucose transmembrane transport",
  "term_id": "GO:1904659",
  "gene_symbol": "SLC2A12"
}